{
  "term_id": "UNKNOWN:0002",
  "gene_name": "Complement C1q tumor necrosis factor-related protein 1",
  "term_label": "Unknown biological process",
  "gene_symbol": "C1QTNF1",
  "gene": "UniProtKB:Q9BXJ1"
}